{
  "gene": "UniProtKB:Q09019",
  "term_label": "deubiquitinase activator activity",
  "gene_symbol": "DMWD",
  "gene_name": "Dystrophia myotonica WD repeat-containing protein",
  "term_id": "GO:0035800"
}